{
  "term_label": "microtubule",
  "gene": "UniProtKB:Q3ZCM7",
  "gene_name": "Tubulin beta-8 chain",
  "gene_symbol": "TUBB8",
  "term_id": "GO:0005874"
}